{
  "term_id": "GO:0004984",
  "gene_symbol": "OR52A5",
  "gene": "UniProtKB:Q9H2C5",
  "term_label": "olfactory receptor activity",
  "gene_name": "Olfactory receptor 52A5"
}